{
  "term_label": "cytoplasmic vesicle",
  "gene_symbol": "HAP1",
  "gene_name": "Huntingtin-associated protein 1",
  "term_id": "GO:0031410",
  "gene": "UniProtKB:P54257"
}